{
  "gene_symbol": "STMN4",
  "term_label": "cytoplasm",
  "term_id": "GO:0005737",
  "gene": "UniProtKB:Q9H169",
  "gene_name": "Stathmin-4"
}